{
  "gene_name": "Syntaxin-binding protein 5-like",
  "term_label": "myosin II binding",
  "term_id": "GO:0045159",
  "gene": "UniProtKB:Q9Y2K9",
  "gene_symbol": "STXBP5L"
}